CD19-Vav-PIK3R1 complex [GO:0070024] (CC) Relationships: is a type of GO:0098797 Definition: A protein complex that contains the cell surface signaling molecule CD19, the Ras guanine nucleotide exchange factor Vav, and the regulatory subunit alpha of phosphatidylinositol 3-kinase (PI3K). References: PMID:7528218 Also known as: CD19-Vav-PI 3-kinase (p85 subunit) complex